{
  "term_id": "GO:0101020",
  "gene_symbol": "CYP3A5",
  "gene": "UniProtKB:P20815",
  "term_label": "estrogen 16-alpha-hydroxylase activity",
  "gene_name": "Cytochrome P450 3A5"
}